mitochondrial DNA-directed RNA polymerase complex [GO:0034245] (cellular component) Relationships: is_a GO:0000428; is a type of GO:0098798 Also known as: mitochondrial RNA polymerase complex, mitochondrial RNA polymerase holoenzyme complex Definition: A DNA-directed RNA polymerase complex located in the mitochondrion. Mitochondrial RNA polymerase is composed of two subunits, a catalytic core, which resembles the enzymes from bacteriophage T7 and T3, and a specificity factor required for promoter recognition, which is similar to members of the eubacterial sigma factor family. In S. cerevisiae, these are encoded by the nuclear genes RPO41 and MTF1 and the specificity factor, required for promoter recognition and initiation, is not present in the elongating form. References: PMID:7929382 Sources: GOC:krc, GOC:mah